{
  "term_id": "GO:0030199",
  "gene_symbol": "LOXL2",
  "gene_name": "Lysyl oxidase homolog 2",
  "term_label": "collagen fibril organization",
  "gene": "UniProtKB:Q9Y4K0"
}